{
  "term_id": "GO:0005634",
  "term_label": "nucleus",
  "gene_name": "Homeobox protein OTX1",
  "gene_symbol": "OTX1",
  "gene": "UniProtKB:P32242"
}